{
  "term_label": "nucleus",
  "gene_name": "Protein SET",
  "term_id": "GO:0005634",
  "gene": "UniProtKB:Q01105",
  "gene_symbol": "SET"
}